mesencephalic trigeminal nucleus development [GO:0021739] (biological process) Definition: The process whose specific outcome is the progression of the mesencephalic trigeminal nucleus over time, from its formation to the mature structure. Sources: GOC:cls, GOC:curators, GOC:dgh, GOC:dph, GOC:jid Relationships: is a type of GO:0021730